{
  "gene_name": "Putative zinc finger protein 730",
  "term_id": "GO:0006355",
  "gene_symbol": "ZNF730",
  "gene": "UniProtKB:Q6ZMV8",
  "term_label": "regulation of DNA-templated transcription"
}